{
  "gene": "UniProtKB:Q8IVT2",
  "gene_name": "Mitotic interactor and substrate of PLK1",
  "term_id": "UNKNOWN:0001",
  "term_label": "Unknown molecular function",
  "gene_symbol": "MISP"
}